{
  "gene_symbol": "SLC13A3",
  "term_id": "GO:0017153",
  "term_label": "sodium:dicarboxylate symporter activity",
  "gene_name": "Na(+)_dicarboxylate cotransporter 3",
  "gene": "UniProtKB:Q8WWT9"
}